kappa-type opioid receptor binding [GO:0031851] (MF) Also known as: kappa-type opioid receptor ligand, dynorphin receptor binding Sources: GOC:mah, GOC:nln Relationships: is a type of GO:0031628 Definition: Binding to a kappa-type opioid receptor.